miRNA-mediated post-transcriptional gene silencing [GO:0035195] (biological process) Relationships: is a type of regulatory ncRNA-mediated post-transcriptional gene silencing [GO:0035194] Also known as: miRNA-mediated gene silencing, gene silencing by miRNA, gene silencing by microRNA, microRNA-mediated gene silencing References: PMID:14744438, PMID:15066275, PMID:15066283, PMID:23209154, PMID:23985560, PMID:28379604 Sources: GOC:aruk, GOC:bc, GOC:rl Subtypes: GO:0035278, miRNA-mediated gene silencing by mRNA destabilization [GO:0035279] Definition: A post-transcriptional gene silencing pathway in which regulatory microRNAs (miRNAs) elicit silencing of specific target genes. miRNAs are endogenous 21-24 nucleotide small RNAs processed from stem-loop RNA precursors (pre-miRNAs). Once incorporated into a RNA-induced silencing complex (RISC), miRNAs can downregulate protein production by either of two posttranscriptional mechanisms: endonucleolytic cleavage of the RNA (often mRNA) or mRNA translational repression, usually accompanied by poly-A tail shortening and subsequent degradation of the mRNA. miRNAs are present in all the animals and in plants, whereas siRNAs are present in lower animals and in plants. Regulation: regulated by GO:0060964; negatively regulated by negative regulation of miRNA-mediated gene silencing [GO:0060965]; positively regulated by positive regulation of miRNA-mediated gene silencing [GO:2000637]